positive regulation of reproductive process [GO:2000243] (biological process) Definition: Any process that activates or increases the frequency, rate or extent of reproductive process. Subtypes: positive regulation of flower development [GO:0009911], positive regulation of conjugation with cellular fusion [GO:0031139], positive regulation of mating type switching [GO:0031496], positive regulation of cumulus cell differentiation [GO:0045594], positive regulation of embryo sac egg cell differentiation [GO:0045696], GO:0045702, GO:0045850, positive regulation of female pigmentation [GO:0048091], GO:0048093, positive regulation of meiotic cell cycle [GO:0051446], GO:0060279, GO:0060282, positive regulation of penile erection [GO:0060406], positive regulation of cortical granule exocytosis by positive regulation of cytosolic calcium ion concentration [GO:0060472], prostate induction [GO:0060514], positive regulation of epithelial cell proliferation involved in prostate gland development [GO:0060769], positive regulation of floral organ abscission [GO:0060861], GO:0070804, GO:0070807, positive regulation of Hulle cell development [GO:0070810], positive regulation of spore-bearing organ development [GO:0075261], positive regulation of anther dehiscence [GO:0120195], positive regulation of oocyte karyosome formation [GO:0120315], positive regulation of regulation of ascospore wall (1->3)-beta-D-glucan biosynthetic process [GO:0140748], GO:1900195, positive regulation of egg-laying behavior [GO:1901046], positive regulation of trophoblast cell migration [GO:1901165], GO:1902040, positive regulation of flagellated sperm motility [GO:1902093], GO:1902437, positive regulation of sperm capacitation [GO:1902492], positive regulation of meiotic DNA double-strand break formation [GO:1903343], positive regulation of asexual reproduction [GO:1903666], positive regulation of maternal process involved in parturition [GO:1904303], positive regulation of establishment of Sertoli cell barrier [GO:1904446], positive regulation of initiation of premeiotic DNA replication [GO:1904514], positive regulation of spindle attachment to meiosis I kinetochore [GO:1904968], positive regulation of synaptonemal complex assembly [GO:1905088], positive regulation of meiotic chromosome separation [GO:1905134], GO:1905326, positive regulation of amoeboid sperm motility [GO:1905418], GO:1905516, positive regulation of oogenesis [GO:1905881], positive regulation of gonad development [GO:1905941], positive regulation of FtsZ-dependent cytokinesis [GO:2000246], GO:2000256, positive regulation of acrosome reaction [GO:2000344], positive regulation of acrosomal vesicle exocytosis [GO:2000368], positive regulation of antral ovarian follicle growth [GO:2000388], positive regulation of seed maturation [GO:2000693] Relationships: is a type of positive regulation of biological process [GO:0048518]; is a type of GO:2000241; positively regulates reproductive process [GO:0022414] Sources: GOC:mah